{
  "term_label": "delayed rectifier potassium channel activity",
  "gene_name": "Potassium voltage-gated channel subfamily A member 3",
  "gene_symbol": "KCNA3",
  "gene": "UniProtKB:P22001",
  "term_id": "GO:0005251"
}